{
  "gene_name": "Unconventional myosin-Id",
  "gene_symbol": "MYO1D",
  "term_label": "actin filament-based movement",
  "term_id": "GO:0030048",
  "gene": "UniProtKB:O94832"
}